{
  "term_label": "sialic acid binding",
  "term_id": "GO:0033691",
  "gene_symbol": "SIGLEC16",
  "gene": "UniProtKB:A6NMB1",
  "gene_name": "Sialic acid-binding Ig-like lectin 16"
}